{
  "gene": "UniProtKB:Q13043",
  "gene_name": "Serine_threonine-protein kinase 4",
  "gene_symbol": "STK4",
  "term_id": "GO:0005737",
  "term_label": "cytoplasm"
}